{
  "term_id": "GO:0003729",
  "term_label": "mRNA binding",
  "gene_name": "Splicing factor 1",
  "gene": "UniProtKB:Q15637",
  "gene_symbol": "SF1"
}